inhibin complex [GO:0043511] (cellular component) Definition: Heterodimeric hormone composed of an inhibin alpha subunit complexed with either an inhibin beta-A subunit, to form inhibin A, or an inhibin beta-B subunit, to form inhibin B. Sources: GOC:jl Note: Note that the actions of the inhibin complex are the opposite of those of the activin complex, which is a dimer of an inhibin beta-A and/or inhibin beta-B subunit. See also the cellular component term 'activin complex ; GO:0048180'. Relationships: is a type of GO:0032991; is part of extracellular space [GO:0005615] Subtypes: inhibin A complex [GO:0043512], GO:0043513